{
  "gene_name": "Dual specificity mitogen-activated protein kinase kinase 1",
  "gene_symbol": "MAP2K1",
  "term_id": "GO:0004708",
  "term_label": "MAP kinase kinase activity",
  "gene": "UniProtKB:Q02750"
}